{
  "gene": "UniProtKB:Q12996",
  "term_id": "GO:0005634",
  "term_label": "nucleus",
  "gene_symbol": "CSTF3",
  "gene_name": "Cleavage stimulation factor subunit 3"
}